{
  "term_label": "spliceosomal snRNP assembly",
  "gene_symbol": "COIL",
  "term_id": "GO:0000387",
  "gene": "UniProtKB:P38432",
  "gene_name": "Coilin"
}